{
  "gene_name": "Protein Spindly",
  "gene": "UniProtKB:Q96EA4",
  "term_id": "GO:0043515",
  "term_label": "kinetochore binding",
  "gene_symbol": "SPDL1"
}